{
  "gene": "UniProtKB:P11844",
  "term_id": "GO:0007601",
  "term_label": "visual perception",
  "gene_symbol": "CRYGA",
  "gene_name": "Gamma-crystallin A"
}